{
  "term_label": "adenylate cyclase-activating adrenergic receptor signaling pathway",
  "term_id": "GO:0071880",
  "gene": "UniProtKB:P35348",
  "gene_symbol": "ADRA1A",
  "gene_name": "Alpha-1A adrenergic receptor"
}